{
  "term_id": "GO:0015631",
  "gene_name": "Tubulin polyglutamylase TTLL6",
  "term_label": "tubulin binding",
  "gene_symbol": "TTLL6",
  "gene": "UniProtKB:Q8N841"
}